ABC-type tungstate transporter activity [GO:1901238] (molecular function) Relationships: is a type of ABC-type transporter activity [GO:0140359] Also known as: tungstate transmembrane transporter activity, ATPase-coupled tungstate transmembrane transporter activity, tungstate transmembrane-transporting ATPase activity Definition: Enables the transfer of a solute or solutes from one side of a membrane to the other according to the reaction: ATP + H2O + tungstate(in) = ADP + phosphate + tungstate(out). References: PMID:16952940, PMID:21784948 Sources: GOC:TermGenie, RHEA:35027